negative regulation of nucleotide-binding domain, leucine rich repeat containing receptor signaling pathway [GO:0070425] (biological process) Definition: Any process that stops, prevents, or reduces the frequency, rate, or extent of a nucleotide-binding domain, leucine rich repeat containing receptor signaling pathway (NLR) pathway. Subtypes: GO:0070429, GO:0070433 Also known as: negative regulation of NOD signaling pathway, negative regulation of nucleotide-binding oligomerization domain containing signaling pathway, negative regulation of nucleotide-binding oligomerization domain containing signalling pathway Sources: GOC:add Relationships: is a type of negative regulation of cytoplasmic pattern recognition receptor signaling pathway [GO:0039532]; is a type of regulation of nucleotide-binding domain, leucine rich repeat containing receptor signaling pathway [GO:0070424]; negatively regulates GO:0035872